directional guidance of interneurons involved in migration from the subpallium to the cortex [GO:0021840] (biological process) Relationships: is a type of regulation of cell migration [GO:0030334]; is part of interneuron migration from the subpallium to the cortex [GO:0021830] Definition: The creation and reception of signals that control the direction of migration of interneurons as a component of the process of migration from the subpallium to the cortex. References: PMID:12626695 Sources: GOC:cls, GOC:dgh, GOC:dph, GOC:jid, GO_REF:0000021